rhamnose transmembrane transport [GO:0015762] (biological process) Also known as: rhamnose transport Relationships: is a type of hexose transmembrane transport [GO:0008645] Definition: The process in which rhamnose is transported across a lipid bilayer, from one side of a membrane to the other. Rhamnose occurs commonly as a compound of plant glycosides, in polysaccharides of gums and mucilages, and in bacterial polysaccharides. It is also a component of some plant cell wall polysaccharides and frequently acts as the sugar components of flavonoids. Sources: GOC:ai